organic acid catabolic process [GO:0016054] (BP) Sources: ISBN:0198506732 Definition: The chemical reactions and pathways resulting in the breakdown of organic acids, any acidic compound containing carbon in covalent linkage. Also known as: organic acid breakdown, organic acid catabolism, organic acid degradation Relationships: is a type of organic acid metabolic process [GO:0006082]; is_a small molecule catabolic process [GO:0044282] Subtypes: 2-aminobenzenesulfonate catabolic process [GO:0046230], toluene-4-sulfonate catabolic process [GO:0046269], alkanesulfonate catabolic process [GO:0046306], GO:0046395, 6-sulfoquinovose(1-) catabolic process [GO:1902777]